{
  "term_id": "GO:0000978",
  "term_label": "RNA polymerase II cis-regulatory region sequence-specific DNA binding",
  "gene_symbol": "TFE3",
  "gene_name": "Transcription factor E3",
  "gene": "UniProtKB:P19532"
}